phosphodiesterase decapping endonuclease activity [GO:1990174] (MF) Definition: Catalysis of the removal of the cap from an unmethylated 5'-end capped RNA resulting in the release of the entire cap structure (GpppN) and a 5' monophosphorylated RNA. References: PMID:20802481 Sources: GOC:dgf Also known as: G(5')pppN pyrophosphatase activity Relationships: is a type of GO:0016891